{
  "gene_symbol": "AMZ1",
  "term_id": "UNKNOWN:0001",
  "gene": "UniProtKB:Q400G9",
  "gene_name": "Archaemetzincin-1",
  "term_label": "Unknown molecular function"
}